N-terminal peptidyl-lysine acetylation [GO:0018076] (BP) Definition: The acetylation of the N-terminal lysine of proteins. Sources: GOC:ai Relationships: is a type of N-terminal protein amino acid acetylation [GO:0006474]; is a type of peptidyl-lysine acetylation [GO:0018394] Regulation: regulated by regulation of N-terminal peptidyl-lysine acetylation [GO:2000759]; RO_0002212 by negative regulation of N-terminal peptidyl-lysine acetylation [GO:2000760]; positively regulated by positive regulation of N-terminal peptidyl-lysine acetylation [GO:2000761]